{
  "gene": "UniProtKB:Q9P2N5",
  "gene_symbol": "RBM27",
  "gene_name": "RNA-binding protein 27",
  "term_id": "GO:0005634",
  "term_label": "nucleus"
}